{
  "gene": "UniProtKB:Q9UFH2",
  "gene_name": "Dynein axonemal heavy chain 17",
  "term_id": "GO:0005930",
  "term_label": "axoneme",
  "gene_symbol": "DNAH17"
}